regulation of actin filament-based process [GO:0032970] (biological process) Subtypes: GO:0032956, regulation of actin filament-based movement [GO:1903115], regulation of actin filament severing [GO:1903918] Definition: Any process that modulates the frequency, rate or extent of any cellular process that depends upon or alters the actin cytoskeleton. Sources: GOC:mah Relationships: is a type of regulation of cellular process [GO:0050794]; regulates actin filament-based process [GO:0030029]